5-hydroxy-L-tryptophan decarboxylase activity [GO:0036467] (molecular function) Sources: GOC:PARL, GOC:bf, RHEA:18533 Also known as: 5-hydroxytryptophan decarboxylase activity Definition: Catalysis of the reaction: 5-hydroxy-L-tryptophan + H+ = CO2 + serotonin. Relationships: is a type of aromatic-L-amino-acid decarboxylase activity [GO:0004058]